{
  "gene": "UniProtKB:P17661",
  "gene_symbol": "DES",
  "gene_name": "Desmin",
  "term_id": "GO:0005882",
  "term_label": "intermediate filament"
}